{
  "term_label": "Unknown molecular function",
  "gene": "UniProtKB:P62945",
  "gene_symbol": "RPL41",
  "gene_name": "Large ribosomal subunit protein eL41",
  "term_id": "UNKNOWN:0001"
}